{
  "term_label": "Golgi cis cisterna",
  "gene_symbol": "GOLGA8M",
  "term_id": "GO:0000137",
  "gene": "UniProtKB:H3BSY2",
  "gene_name": "Golgin subfamily A member 8M"
}